{
  "term_label": "negative regulation of epidermal growth factor receptor signaling pathway",
  "gene": "UniProtKB:Q9UJM3",
  "gene_symbol": "ERRFI1",
  "gene_name": "ERBB receptor feedback inhibitor 1",
  "term_id": "GO:0042059"
}